{
  "gene_name": "STEAP family member 1B",
  "term_id": "GO:0005886",
  "gene": "UniProtKB:Q6NZ63",
  "term_label": "plasma membrane",
  "gene_symbol": "STEAP1B"
}